carbohydrate catabolic process [GO:0016052] (biological process) Definition: The chemical reactions and pathways resulting in the breakdown of carbohydrates, any of a group of organic compounds based of the general formula Cx(H2O)y. Sources: ISBN:0198506732 Also known as: carbohydrate breakdown, carbohydrate catabolism, carbohydrate degradation, catabolic carbohydrate metabolic process, catabolic carbohydrate metabolism, multicellular organismal carbohydrate catabolic process, single-organism carbohydrate catabolic process Relationships: is a type of carbohydrate metabolic process [GO:0005975]; is a type of catabolic process [GO:0009056] Subtypes: GO:0000272, glycolytic process [GO:0006096], oligosaccharide catabolic process [GO:0009313], GO:0019405, GO:0034194, L-galactonate catabolic process [GO:0034195], D-glucarate catabolic process [GO:0042838], L-idonate catabolic process [GO:0046183], monosaccharide catabolic process [GO:0046365], Entner-Doudoroff pathway [GO:0061678], L-altrarate catabolic process [GO:1903663] Regulation: regulated by regulation of carbohydrate catabolic process [GO:0043470]